{
  "term_id": "GO:0005634",
  "gene_name": "Inactive ubiquitin carboxyl-terminal hydrolase 17-like protein 7",
  "term_label": "nucleus",
  "gene_symbol": "USP17L7",
  "gene": "UniProtKB:P0C7H9"
}